{
  "term_id": "UNKNOWN:0003",
  "gene_name": "UPF0538 protein C2orf76",
  "gene_symbol": "C2orf76",
  "gene": "UniProtKB:Q3KRA6",
  "term_label": "Unknown cellular component"
}